{
  "gene": "UniProtKB:O15399",
  "term_id": "GO:0005886",
  "gene_name": "Glutamate receptor ionotropic, NMDA 2D",
  "gene_symbol": "GRIN2D",
  "term_label": "plasma membrane"
}